{
  "term_label": "RNA processing",
  "term_id": "GO:0006396",
  "gene_symbol": "ADARB2",
  "gene": "UniProtKB:Q9NS39",
  "gene_name": "Double-stranded RNA-specific editase B2"
}